{
  "term_label": "cytoplasm",
  "term_id": "GO:0005737",
  "gene": "UniProtKB:Q5SWL8",
  "gene_name": "PRAME family member 19",
  "gene_symbol": "PRAMEF19"
}